superior salivary nucleus development [GO:0021753] (biological process) Relationships: is a type of GO:0021751 Sources: GOC:cls, GOC:curators, GOC:dgh, GOC:dph, GOC:jid Definition: The process whose specific outcome is the progression of the superior salivary nucleus over time, from its formation to the mature structure.